chloroplast vesicle [GO:0062247] (cellular component) Definition: A intracellular vesicle that is part of a chloroplast. References: PMID:32245810 Relationships: is a type of cytoplasmic vesicle [GO:0031410]; is part of chloroplast [GO:0009507]